regulation of muscle filament sliding speed [GO:0032972] (biological process) Sources: GOC:dph, GOC:ecd, GOC:tb Relationships: is a type of regulation of muscle filament sliding [GO:0032971]; is a type of GO:0065008 Definition: Any process that modulates the velocity of muscle filament sliding. Subtypes: GO:0014915